{
  "gene_name": "Immunoglobulin heavy variable 3_OR16-8 (non-functional) (Fragment)",
  "gene": "UniProtKB:A0A075B7F1",
  "gene_symbol": "IGHV3OR16-8",
  "term_label": "Unknown cellular component",
  "term_id": "UNKNOWN:0003"
}